{
  "gene_symbol": "WNT5B",
  "gene_name": "Protein Wnt-5b",
  "term_id": "GO:0030182",
  "gene": "UniProtKB:Q9H1J7",
  "term_label": "neuron differentiation"
}